{
  "gene_name": "PDZ and LIM domain protein 3",
  "gene_symbol": "PDLIM3",
  "gene": "UniProtKB:Q53GG5",
  "term_id": "GO:0030018",
  "term_label": "Z disc"
}